negative regulation of indoleacetic acid biosynthetic process via tryptophan [GO:1901997] (biological process) Also known as: down regulation of IAA biosynthetic process via tryptophan, down regulation of indoleacetic acid anabolism via tryptophan, down regulation of indoleacetic acid biosynthetic process via tryptophan, down regulation of indoleacetic acid formation via tryptophan, down regulation of indoleacetic acid synthesis via tryptophan, down-regulation of IAA biosynthetic process via tryptophan, down-regulation of indoleacetic acid anabolism via tryptophan, down-regulation of indoleacetic acid biosynthetic process via tryptophan, down-regulation of indoleacetic acid formation via tryptophan, down-regulation of indoleacetic acid synthesis via tryptophan, downregulation of IAA biosynthetic process via tryptophan, downregulation of indoleacetic acid anabolism via tryptophan, downregulation of indoleacetic acid biosynthetic process via tryptophan, downregulation of indoleacetic acid formation via tryptophan, downregulation of indoleacetic acid synthesis via tryptophan, inhibition of IAA biosynthetic process via tryptophan, inhibition of indoleacetic acid anabolism via tryptophan, inhibition of indoleacetic acid formation via tryptophan, inhibition of indoleacetic acid synthesis via tryptophan, negative regulation of IAA biosynthetic process via tryptophan, negative regulation of indoleacetic acid anabolism via tryptophan, negative regulation of indoleacetic acid formation via tryptophan, negative regulation of indoleacetic acid synthesis via tryptophan, inhibition of indoleacetic acid biosynthetic process via tryptophan References: PMID:23377040 Sources: GOC:TermGenie Relationships: is a type of negative regulation of hormone biosynthetic process [GO:0032353]; is a type of negative regulation of amino acid metabolic process [GO:0045763]; is a type of GO:0062014; is a type of GO:0090356; is a type of regulation of indoleacetic acid biosynthetic process via tryptophan [GO:1901996]; negatively regulates indoleacetic acid biosynthetic process via tryptophan [GO:0009848] Definition: Any process that stops, prevents or reduces the frequency, rate or extent of indoleacetic acid biosynthetic process via tryptophan.